positive regulation of activin secretion [GO:0032337] (biological process) Sources: GOC:mah Also known as: up regulation of activin secretion, up-regulation of activin secretion, upregulation of activin secretion, activation of activin secretion, stimulation of activin secretion Definition: Any process that activates or increases the frequency, rate or extent of the regulated release of activin from a cell. Relationships: is a type of regulation of activin secretion [GO:0032335]; is a type of positive regulation of hormone secretion [GO:0046887]; positively regulates activin secretion [GO:0032333]